effector-mediated suppression of host defense response [GO:0140590] (biological process) Relationships: is a type of effector-mediated perturbation of host defenses by symbiont [GO:0140415] Definition: A process mediated by a molecule secreted by a symbiont that results in the suppression of a defense response. The host is defined as the larger of the organisms involved in a symbiotic interaction. Also known as: effector-mediated suppression of host defenses by symbiont, effector-mediated suppression of host defenses Subtypes: effector-mediated suppression of host innate immune response [GO:0140403] References: PMID:28082413